{
  "term_id": "GO:0000398",
  "gene_name": "RNA-binding motif protein, Y chromosome, family 1 member A1",
  "gene": "UniProtKB:P0DJD3",
  "term_label": "mRNA splicing, via spliceosome",
  "gene_symbol": "RBMY1A1"
}